{
  "gene_name": "Keratin-associated protein 29-1",
  "term_id": "UNKNOWN:0001",
  "gene_symbol": "KRTAP29-1",
  "gene": "UniProtKB:A8MX34",
  "term_label": "Unknown molecular function"
}